{
  "gene_name": "Tripartite motif-containing protein 49D",
  "gene_symbol": "TRIM49D1",
  "term_label": "cytoplasm",
  "term_id": "GO:0005737",
  "gene": "UniProtKB:C9J1S8"
}